{
  "gene": "UniProtKB:O94819",
  "term_id": "UNKNOWN:0001",
  "gene_name": "Kelch repeat and BTB domain-containing protein 11",
  "term_label": "Unknown molecular function",
  "gene_symbol": "KBTBD11"
}